{
  "gene": "UniProtKB:Q05209",
  "term_id": "GO:0005634",
  "term_label": "nucleus",
  "gene_symbol": "PTPN12",
  "gene_name": "Tyrosine-protein phosphatase non-receptor type 12"
}